{
  "term_label": "Unknown cellular component",
  "gene_name": "Actin-histidine N-methyltransferase",
  "gene": "UniProtKB:Q86TU7",
  "gene_symbol": "SETD3",
  "term_id": "UNKNOWN:0003"
}